{
  "gene_symbol": "BBS9",
  "gene": "UniProtKB:Q3SYG4",
  "term_label": "membrane",
  "gene_name": "Protein PTHB1",
  "term_id": "GO:0016020"
}